{
  "gene_name": "Ankyrin repeat domain-containing protein 34A",
  "gene_symbol": "ANKRD34A",
  "term_label": "pi-body",
  "gene": "UniProtKB:Q69YU3",
  "term_id": "GO:0071546"
}